{
  "term_id": "GO:0005509",
  "gene_name": "Myosin regulatory light chain 11",
  "gene_symbol": "MYL11",
  "term_label": "calcium ion binding",
  "gene": "UniProtKB:Q96A32"
}